{
  "term_id": "GO:0005634",
  "gene": "UniProtKB:Q14997",
  "term_label": "nucleus",
  "gene_name": "Proteasome activator complex subunit 4",
  "gene_symbol": "PSME4"
}